{
  "gene_name": "KAT8 regulatory NSL complex subunit 1",
  "term_id": "GO:0035035",
  "gene_symbol": "KANSL1",
  "gene": "UniProtKB:Q7Z3B3",
  "term_label": "histone acetyltransferase binding"
}